calcium ion import across plasma membrane [GO:0098703] (biological process) Definition: The directed movement of calcium ions from outside of a cell, across the plasma membrane and into the cytosol. Sources: GOC:dos Relationships: is a type of GO:0070509; is_a GO:0097553; is a type of inorganic cation import across plasma membrane [GO:0098659]; is a type of GO:1902656 Also known as: calcium ion import into cell, calcium ion uptake into cell Regulation: regulated by regulation of calcium ion import across plasma membrane [GO:1905664]; positively regulated by GO:1905665; negatively regulated by negative regulation of calcium ion import across plasma membrane [GO:1905949]